dGTP metabolic process [GO:0046070] (biological process) Definition: The chemical reactions and pathways involving dGTP, guanosine triphosphate. Sources: GOC:go_curators Also known as: dGTP metabolism Relationships: is a type of purine deoxyribonucleotide metabolic process [GO:0009151]; is a type of purine deoxyribonucleoside triphosphate metabolic process [GO:0009215] Subtypes: dGTP catabolic process [GO:0006203], dGTP biosynthetic process [GO:0046071]